{
  "term_id": "UNKNOWN:0001",
  "gene_name": "Uncharacterized protein FLJ46757",
  "gene_symbol": "Q6ZR03",
  "term_label": "Unknown molecular function",
  "gene": "UniProtKB:Q6ZR03"
}